{
  "term_label": "Unknown cellular component",
  "gene_symbol": "TRAV13-1",
  "gene": "UniProtKB:A0A0B4J241",
  "term_id": "UNKNOWN:0003",
  "gene_name": "T cell receptor alpha variable 13-1"
}